{
  "gene_symbol": "ATP1A1",
  "gene": "UniProtKB:P05023",
  "term_label": "potassium ion import across plasma membrane",
  "gene_name": "Sodium_potassium-transporting ATPase subunit alpha-1",
  "term_id": "GO:1990573"
}